{
  "term_label": "Unknown biological process",
  "gene_symbol": "FAM180B",
  "gene": "UniProtKB:Q6P0A1",
  "gene_name": "Protein FAM180B",
  "term_id": "UNKNOWN:0002"
}